{
  "gene_symbol": "GRXCR2",
  "term_label": "Unknown molecular function",
  "gene": "UniProtKB:A6NFK2",
  "gene_name": "Glutaredoxin domain-containing cysteine-rich protein 2",
  "term_id": "UNKNOWN:0001"
}